{
  "gene": "UniProtKB:P09919",
  "gene_symbol": "CSF3",
  "gene_name": "Granulocyte colony-stimulating factor",
  "term_label": "macrophage differentiation",
  "term_id": "GO:0030225"
}